{
  "term_id": "GO:0000381",
  "term_label": "regulation of alternative mRNA splicing, via spliceosome",
  "gene": "UniProtKB:Q96PK6",
  "gene_symbol": "RBM14",
  "gene_name": "RNA-binding protein 14"
}